{
  "gene_name": "MAL-like protein",
  "gene_symbol": "MALL",
  "term_label": "myelination",
  "gene": "UniProtKB:Q13021",
  "term_id": "GO:0042552"
}